hydrogen peroxide-mediated programmed cell death [GO:0010421] (biological process) Also known as: programmed cell death in response to hydrogen peroxide References: PMID:16036580 Sources: GOC:mtg_apoptosis Definition: Programmed cell death induced by hydrogen peroxide. Programmed cell death is the cell death resulting from activation of endogenous cellular processes. Regulation: regulated by GO:1901298; RO_0002212 by negative regulation of hydrogen peroxide-mediated programmed cell death [GO:1901299]; positively regulated by positive regulation of hydrogen peroxide-mediated programmed cell death [GO:1901300] Relationships: is a type of programmed cell death in response to reactive oxygen species [GO:0097468]